{
  "gene": "UniProtKB:Q9NP87",
  "gene_symbol": "POLM",
  "gene_name": "DNA-directed DNA_RNA polymerase mu",
  "term_id": "GO:0006303",
  "term_label": "double-strand break repair via nonhomologous end joining"
}